{
  "term_label": "ceramide transport",
  "gene_name": "Glycolipid transfer protein domain-containing protein 2",
  "gene": "UniProtKB:A6NH11",
  "gene_symbol": "GLTPD2",
  "term_id": "GO:0035627"
}